isomerase activity [GO:0016853] (molecular function) Subtypes: racemase and epimerase activity [GO:0016854], cis-trans isomerase activity [GO:0016859], intramolecular oxidoreductase activity [GO:0016860], intramolecular transferase activity [GO:0016866], intramolecular lyase activity [GO:0016872], GO:0051075, peroxynitrite isomerase activity [GO:0062213], GO:0120543 Sources: ISBN:0198506732 Also known as: other isomerase activity Relationships: is a type of catalytic activity [GO:0003824] Definition: Catalysis of the geometric or structural changes within one molecule. Isomerase is the systematic name for any enzyme of EC class 5.